{
  "gene_symbol": "CD1C",
  "term_label": "external side of plasma membrane",
  "term_id": "GO:0009897",
  "gene": "UniProtKB:P29017",
  "gene_name": "T-cell surface glycoprotein CD1c"
}